2-hydroxy-ATP hydrolase activity [GO:0106377] (molecular function) Definition: Catalysis of the reaction: 2-hydroxy-ATP + H2O = 2-hydroxy-AMP + H+ + diphosphate. Relationships: is_a GO:0047429 References: PMID:11139615 Sources: RHEA:67392